{
  "gene_name": "E3 ubiquitin-protein ligase RNF180",
  "term_label": "norepinephrine metabolic process",
  "term_id": "GO:0042415",
  "gene": "UniProtKB:Q86T96",
  "gene_symbol": "RNF180"
}